{
  "term_id": "UNKNOWN:0002",
  "gene_name": "Folliculin-interacting protein 1",
  "gene": "UniProtKB:Q8TF40",
  "gene_symbol": "FNIP1",
  "term_label": "Unknown biological process"
}